{
  "gene_symbol": "ZBTB38",
  "gene_name": "Zinc finger and BTB domain-containing protein 38",
  "gene": "UniProtKB:Q8NAP3",
  "term_label": "RNA polymerase II cis-regulatory region sequence-specific DNA binding",
  "term_id": "GO:0000978"
}